{
  "gene_symbol": "WASF1",
  "gene_name": "Actin-binding protein WASF1",
  "term_label": "Arp2/3 complex binding",
  "gene": "UniProtKB:Q92558",
  "term_id": "GO:0071933"
}